{
  "gene_name": "Rho GTPase-activating protein 44",
  "gene": "UniProtKB:Q17R89",
  "term_label": "dendritic spine",
  "term_id": "GO:0043197",
  "gene_symbol": "ARHGAP44"
}